{
  "gene_symbol": "GGTLC1",
  "gene": "UniProtKB:Q9BX51",
  "gene_name": "Glutathione hydrolase light chain 1",
  "term_label": "Unknown molecular function",
  "term_id": "UNKNOWN:0001"
}